histone H4K8 acetyltransferase activity [GO:0043996] (molecular function) Also known as: histone acetylase activity (H4-K8 specific), histone acetyltransferase activity (H4-K8 specific), histone lysine N-acetyltransferase activity (H4-K8 specific) Relationships: is a type of GO:0010485 References: PMID:18552846, PMID:19056256 Definition: Catalysis of the reaction: acetyl-CoA + histone H4 L-lysine (position 8) = CoA + histone H4 N6-acetyl-L-lysine (position 8). Note: Note that the residue position corresponds to the canonical human H4 histone (UniProtKB:P02309); this residue is conserved across all eukaryotes. Note that the initiation methionine is cleaved, so the first residue is S1.